{
  "gene": "UniProtKB:P01135",
  "term_label": "growth factor activity",
  "gene_name": "Protransforming growth factor alpha",
  "term_id": "GO:0008083",
  "gene_symbol": "TGFA"
}